{
  "term_label": "fatty acid transport",
  "term_id": "GO:0015908",
  "gene": "UniProtKB:P50120",
  "gene_symbol": "RBP2",
  "gene_name": "Retinol-binding protein 2"
}